{
  "gene_name": "Dystrophia myotonica WD repeat-containing protein",
  "term_id": "GO:0005737",
  "gene_symbol": "DMWD",
  "term_label": "cytoplasm",
  "gene": "UniProtKB:Q09019"
}